{
  "term_id": "GO:0044609",
  "gene_name": "DBIRD complex subunit ZNF326",
  "gene": "UniProtKB:Q5BKZ1",
  "term_label": "DBIRD complex",
  "gene_symbol": "ZNF326"
}